micronucleus organization [GO:0032125] (biological process) References: PMID:10503190 Sources: GOC:dph, GOC:jl, GOC:mah Definition: A process that is carried out at the cellular level which results in the assembly, arrangement of constituent parts, or disassembly of the micronucleus. Also known as: micronuclear organization, micronucleus organisation, micronuclear organization and biogenesis Relationships: is a type of nucleus organization [GO:0006997]